{
  "gene": "UniProtKB:Q96KR1",
  "gene_name": "Zinc finger RNA-binding protein",
  "term_id": "GO:0003725",
  "term_label": "double-stranded RNA binding",
  "gene_symbol": "ZFR"
}